{
  "gene": "UniProtKB:A0A0J9YW14",
  "gene_symbol": "IGHJ3",
  "term_label": "Unknown cellular component",
  "gene_name": "Immunoglobulin heavy joining 3 (Fragment)",
  "term_id": "UNKNOWN:0003"
}